{
  "gene_name": "Nuclear RNA export factor 1",
  "term_id": "GO:0003723",
  "term_label": "RNA binding",
  "gene": "UniProtKB:Q9UBU9",
  "gene_symbol": "NXF1"
}